metanephric tubule morphogenesis [GO:0072173] (biological process) Subtypes: metanephric nephron tubule morphogenesis [GO:0072282] Sources: GOC:mtg_kidney_jan10 Relationships: is a type of GO:0060562; is part of metanephric tubule development [GO:0072170] Definition: The process in which the anatomical structures of a metanephric tubule are generated and organized from an epithelium. A metanephric tubule is an epithelial tube that is part of the metanephros.